{
  "term_id": "GO:1990904",
  "gene_symbol": "GRSF1",
  "gene": "UniProtKB:Q12849",
  "gene_name": "G-rich sequence factor 1",
  "term_label": "ribonucleoprotein complex"
}